postsynapse to nucleus signaling pathway [GO:0099527] (biological process) Regulation: regulated by regulation of postsynapse to nucleus signaling pathway [GO:1905539] Also known as: postsynaptic signaling to nucleus References: PMID:24317321, PMID:25652077 Sources: GOC:dos Definition: The series of molecular signals that conveys information from the postsynapse to the nucleus via cytoskeletal transport of a protein from a postsynapse to the component to the nucleus where it affects biochemical processes that occur in the nucleus (e.g DNA transcription, mRNA splicing, or DNA/histone modifications). Relationships: is a type of GO:0098926